{
  "gene": "UniProtKB:Q7Z4V0",
  "gene_name": "Zinc finger protein 438",
  "term_label": "DNA-binding transcription factor activity, RNA polymerase II-specific",
  "gene_symbol": "ZNF438",
  "term_id": "GO:0000981"
}